{
  "gene_name": "Replication protein A 14 kDa subunit",
  "gene_symbol": "RPA3",
  "term_label": "double-strand break repair via homologous recombination",
  "term_id": "GO:0000724",
  "gene": "UniProtKB:P35244"
}